{
  "gene_symbol": "ATP2C2",
  "gene_name": "Calcium-transporting ATPase type 2C member 2",
  "term_label": "intracellular calcium ion homeostasis",
  "gene": "UniProtKB:O75185",
  "term_id": "GO:0006874"
}